{
  "term_label": "endoplasmic reticulum",
  "gene_symbol": "ATP11A",
  "gene": "UniProtKB:P98196",
  "term_id": "GO:0005783",
  "gene_name": "Phospholipid-transporting ATPase IH"
}